{
  "gene_name": "Blood group Rh(CE) polypeptide",
  "gene_symbol": "RHCE",
  "term_id": "GO:0008519",
  "gene": "UniProtKB:P18577",
  "term_label": "ammonium channel activity"
}